{
  "gene_symbol": "KLHL24",
  "gene_name": "Kelch-like protein 24",
  "term_id": "GO:1990756",
  "term_label": "ubiquitin-like ligase-substrate adaptor activity",
  "gene": "UniProtKB:Q6TFL4"
}